{
  "gene_symbol": "TMX1",
  "gene": "UniProtKB:Q9H3N1",
  "gene_name": "Thioredoxin-related transmembrane protein 1",
  "term_label": "endomembrane system",
  "term_id": "GO:0012505"
}